cis-3,4-dihydrophenanthrene-3,4-diol dehydrogenase activity [GO:0018507] (molecular function) Relationships: is a type of GO:0016628 Definition: Catalysis of the reaction: (3S,4R)-3,4-dihydrophenanthrene-3,4-diol + NAD+ = H+ + NADH + phenanthrene-3,4-diol. Also known as: cis-3,4-dihydroxy-3,4-dihydrophenanthrene dehydrogenase activity, (+)-cis-3,4-dihydrophenanthrene-3,4-diol:NAD+ 3,4-oxidoreductase activity Sources: EC:1.3.1.49, RHEA:16253